fructose binding [GO:0070061] (molecular function) Definition: Binding to the D- or L-enantiomer of fructose, the ketohexose arabino-hex-2-ulose. Sources: CHEBI:28757, GOC:BHF, GOC:mah Relationships: is a type of monosaccharide binding [GO:0048029]